{
  "gene_symbol": "EXOSC10",
  "term_label": "histone mRNA catabolic process",
  "term_id": "GO:0071044",
  "gene": "UniProtKB:Q01780",
  "gene_name": "Exosome component 10"
}